{
  "term_label": "Unknown cellular component",
  "gene_symbol": "PKD1L1-AS1",
  "gene": "UniProtKB:Q9H7B7",
  "gene_name": "Putative uncharacterized protein PKD1L1-AS1",
  "term_id": "UNKNOWN:0003"
}